{
  "term_label": "endomembrane system",
  "gene": "UniProtKB:P20340",
  "term_id": "GO:0012505",
  "gene_name": "Ras-related protein Rab-6A",
  "gene_symbol": "RAB6A"
}